{
  "gene_symbol": "BCL2L10",
  "term_label": "intrinsic apoptotic signaling pathway in response to DNA damage",
  "gene": "UniProtKB:Q9HD36",
  "term_id": "GO:0008630",
  "gene_name": "Bcl-2-like protein 10"
}